tropinesterase activity [GO:0050357] (molecular function) Relationships: is a type of carboxylic ester hydrolase activity [GO:0052689] Definition: Catalysis of the reaction: atropine + H2O = H+ + tropate + tropine. Sources: EC:3.1.1.10, RHEA:23304 Also known as: atropinase activity, atropine acylhydrolase activity, atropine esterase activity, atropinesterase activity, tropine esterase activity